{
  "gene_name": "Long-chain-fatty-acid--CoA ligase ACSBG1",
  "gene_symbol": "ACSBG1",
  "gene": "UniProtKB:Q96GR2",
  "term_id": "GO:0042759",
  "term_label": "long-chain fatty acid biosynthetic process"
}